{
  "gene_name": "Keratin-associated protein 19-6",
  "gene": "UniProtKB:Q3LI70",
  "term_label": "Unknown biological process",
  "term_id": "UNKNOWN:0002",
  "gene_symbol": "KRTAP19-6"
}